{
  "gene_name": "Mesencephalic astrocyte-derived neurotrophic factor",
  "gene": "UniProtKB:P55145",
  "term_label": "dopaminergic neuron differentiation",
  "gene_symbol": "MANF",
  "term_id": "GO:0071542"
}